{
  "gene_symbol": "GLDC",
  "gene": "UniProtKB:P23378",
  "term_label": "pyridoxal phosphate binding",
  "gene_name": "Glycine dehydrogenase (decarboxylating), mitochondrial",
  "term_id": "GO:0030170"
}